synaptic vesicle coating [GO:0016183] (biological process) References: PMID:10099709, PMID:20448150 Sources: GOC:curators Definition: The formation of clathrin coated pits in the presynaptic membrane endocytic zone, triggered by the presence of high concentrations of synaptic vesicle components. This process leads to, but does not include budding of the membrane to form new vesicles. Relationships: is a type of vesicle coating [GO:0006901]; is part of synaptic vesicle budding from presynaptic endocytic zone membrane [GO:0016185]